{
  "gene_symbol": "FBXO38",
  "term_label": "SCF-dependent proteasomal ubiquitin-dependent protein catabolic process",
  "gene_name": "F-box only protein 38",
  "gene": "UniProtKB:Q6PIJ6",
  "term_id": "GO:0031146"
}